{
  "term_label": "Unknown molecular function",
  "gene_name": "Cytochrome P450 4B1",
  "term_id": "UNKNOWN:0001",
  "gene_symbol": "CYP4B1",
  "gene": "UniProtKB:P13584"
}